{
  "term_label": "signal transduction",
  "gene_name": "TOM1-like protein 2",
  "term_id": "GO:0007165",
  "gene_symbol": "TOM1L2",
  "gene": "UniProtKB:Q6ZVM7"
}